{
  "gene": "UniProtKB:Q13087",
  "term_label": "response to endoplasmic reticulum stress",
  "term_id": "GO:0034976",
  "gene_symbol": "PDIA2",
  "gene_name": "Protein disulfide-isomerase A2"
}